pheophorbide a oxygenase activity [GO:0032441] (molecular function) Relationships: is a type of GO:0016730 References: PMID:14657372 Definition: Catalysis of the reaction: pheophorbide a + reduced ferredoxin + 2 O2 = red chlorophyll catabolite + oxidized ferredoxin + H2O.